{
  "gene_name": "Melanoma-associated antigen E2",
  "term_label": "Unknown molecular function",
  "gene_symbol": "MAGEE2",
  "term_id": "UNKNOWN:0001",
  "gene": "UniProtKB:Q8TD90"
}